{
  "gene_name": "Oncomodulin-1",
  "term_id": "UNKNOWN:0002",
  "term_label": "Unknown biological process",
  "gene": "UniProtKB:P0CE72",
  "gene_symbol": "OCM"
}